{
  "term_label": "Unknown cellular component",
  "gene_symbol": "RTKN2",
  "term_id": "UNKNOWN:0003",
  "gene_name": "Rhotekin-2",
  "gene": "UniProtKB:Q8IZC4"
}